{
  "gene_symbol": "ZSCAN5C",
  "gene": "UniProtKB:A6NGD5",
  "term_id": "GO:0000978",
  "gene_name": "Zinc finger and SCAN domain-containing protein 5C",
  "term_label": "RNA polymerase II cis-regulatory region sequence-specific DNA binding"
}